{
  "gene_name": "Activating transcription factor 7-interacting protein 1",
  "gene_symbol": "ATF7IP",
  "term_label": "transcription coregulator activity",
  "gene": "UniProtKB:Q6VMQ6",
  "term_id": "GO:0003712"
}